{
  "term_label": "metal ion binding",
  "gene_name": "Metallothionein-1H",
  "term_id": "GO:0046872",
  "gene_symbol": "MT1H",
  "gene": "UniProtKB:P80294"
}